{
  "gene_name": "Neurogenic differentiation factor 1",
  "term_id": "GO:0061564",
  "term_label": "axon development",
  "gene_symbol": "NEUROD1",
  "gene": "UniProtKB:Q13562"
}